{
  "term_label": "intracellular protein transport",
  "gene_name": "Transmembrane emp24 domain-containing protein 5",
  "gene_symbol": "TMED5",
  "term_id": "GO:0006886",
  "gene": "UniProtKB:Q9Y3A6"
}